negative regulation of non-canonical NF-kappaB signal transduction [GO:1901223] (biological process) Sources: GOC:TermGenie Also known as: down regulation of NIK/NF-kappaB cascade, down regulation of non-canonical NF-KB signaling, down regulation of noncanonical NF-kappaB signaling, down regulation of noncanonical nuclear factor kappaB (NF-kappaB) pathway, down-regulation of NIK/NF-kappaB cascade, down-regulation of non-canonical NF-KB signaling, down-regulation of noncanonical NF-kappaB signaling, down-regulation of noncanonical nuclear factor kappaB (NF-kappaB) pathway, downregulation of NIK/NF-kappaB cascade, downregulation of non-canonical NF-KB signaling, downregulation of noncanonical NF-kappaB signaling, downregulation of noncanonical nuclear factor kappaB (NF-kappaB) pathway, inhibition of non-canonical NF-KB signaling, inhibition of noncanonical NF-kappaB signaling, inhibition of noncanonical nuclear factor kappaB (NF-kappaB) pathway, negative regulation of NIK/NF-kappaB cascade, negative regulation of NIK/NF-kappaB signaling, negative regulation of non-canonical NF-KB signaling, negative regulation of noncanonical NF-kappaB signaling, negative regulation of noncanonical nuclear factor kappaB (NF-kappaB) pathway, down regulation of p52-dependent NF-kappaB signaling, down-regulation of p52-dependent NF-kappaB signaling, downregulation of p52-dependent NF-kappaB signaling, inhibition of NIK/NF-kappaB cascade, inhibition of p52-dependent NF-kappaB signaling, negative regulation of NF-kappaB import into nucleus, negative regulation of p52-dependent NF-kappaB signaling Definition: Any process that stops, prevents or reduces the frequency, rate or extent of non-canonical NF-kappaB signaling cascade. Relationships: is a type of GO:1901222; is a type of GO:1902532; negatively regulates GO:0038061